{
  "gene_name": "Gasdermin-C",
  "gene": "UniProtKB:Q9BYG8",
  "term_id": "GO:0042742",
  "gene_symbol": "GSDMC",
  "term_label": "defense response to bacterium"
}